{
  "gene_name": "Meiotic recombination protein DMC1_LIM15 homolog",
  "gene_symbol": "DMC1",
  "gene": "UniProtKB:Q14565",
  "term_label": "DNA recombinase assembly",
  "term_id": "GO:0000730"
}